NEDD8 activating enzyme activity [GO:0019781] (molecular function) Relationships: is a type of ubiquitin-like modifier activating enzyme activity [GO:0008641] Definition: Catalysis of the initiation of the NEDD8 (RUB1) conjugation cascade. References: PMID:12646924 Also known as: RUB1 activating enzyme activity